swim bladder inflation [GO:0048798] (biological process) Also known as: gas bladder inflation Sources: GOC:mh Relationships: is a type of GO:0009653; is part of GO:0048796 Definition: The expansion of the swim bladder by trapped gases. The swim bladder is used by some fishes to maintain buoyancy and may function in addition as a sound producing organ, a sound receptor, and a respiratory organ.